collagen-activated tyrosine kinase receptor signaling pathway [GO:0038063] (biological process) Definition: The series of molecular signals initiated by collagen binding to its receptor on the surface of a target cell where the receptor possesses tyrosine kinase activity, and ending with the regulation of a downstream cellular process, e.g. transcription. References: PMID:15888913, PMID:16626936 Sources: GOC:bf, GOC:uh Relationships: is a type of cell surface receptor protein tyrosine kinase signaling pathway [GO:0007169]; is a type of GO:0038065 Also known as: collagen-activated RTK signaling pathway, collagen-activated tyrosine kinase receptor signalling pathway, DDR signaling pathway, discoidin domain receptor signaling pathway